{
  "term_id": "GO:0000151",
  "gene_name": "DCN1-like protein 2",
  "term_label": "ubiquitin ligase complex",
  "gene": "UniProtKB:Q6PH85",
  "gene_symbol": "DCUN1D2"
}